{
  "gene_symbol": "ANKLE2",
  "gene_name": "Ankyrin repeat and LEM domain-containing protein 2",
  "gene": "UniProtKB:Q86XL3",
  "term_id": "GO:0007084",
  "term_label": "mitotic nuclear membrane reassembly"
}